{
  "term_id": "GO:0005789",
  "term_label": "endoplasmic reticulum membrane",
  "gene": "UniProtKB:O95197",
  "gene_name": "Reticulon-3",
  "gene_symbol": "RTN3"
}